{
  "term_label": "zinc ion transmembrane transporter activity",
  "gene_name": "Zinc transporter ZIP13",
  "gene": "UniProtKB:Q96H72",
  "term_id": "GO:0005385",
  "gene_symbol": "SLC39A13"
}